{
  "gene_name": "Serine_threonine-protein kinase Sgk3",
  "term_label": "Unknown cellular component",
  "term_id": "UNKNOWN:0003",
  "gene_symbol": "SGK3",
  "gene": "UniProtKB:Q96BR1"
}